{
  "term_id": "GO:1904200",
  "term_label": "iodide transmembrane transport",
  "gene_symbol": "SLC5A5",
  "gene_name": "Sodium_iodide cotransporter",
  "gene": "UniProtKB:Q92911"
}